{
  "gene": "UniProtKB:Q86UD1",
  "gene_name": "Out at first protein homolog",
  "gene_symbol": "OAF",
  "term_id": "UNKNOWN:0003",
  "term_label": "Unknown cellular component"
}